{
  "term_label": "membrane",
  "gene": "UniProtKB:Q15646",
  "gene_name": "2'-5'-oligoadenylate synthase-like protein",
  "gene_symbol": "OASL",
  "term_id": "GO:0016020"
}